{
  "term_id": "GO:0002312",
  "gene_name": "Interferon epsilon",
  "gene": "UniProtKB:Q86WN2",
  "gene_symbol": "IFNE",
  "term_label": "B cell activation involved in immune response"
}